{
  "term_id": "GO:0045202",
  "term_label": "synapse",
  "gene": "UniProtKB:Q13425",
  "gene_symbol": "SNTB2",
  "gene_name": "Beta-2-syntrophin"
}